negative regulation of mitotic actomyosin contractile ring contraction [GO:1903472] (biological process) Definition: Any process that stops, prevents or reduces the frequency, rate or extent of mitotic actomyosin contractile ring contraction. References: PMID:1234 Sources: GOC:TermGenie, GOC:mtg_cell_cycle, GO_REF:0000058 Also known as: down regulation of contractile ring contraction involved in cell cycle cytokinesis involved in mitotic cell cycle, down regulation of cytokinesis, actomyosin ring contraction involved in mitotic cell cycle, down regulation of mitotic actomyosin contractile ring contraction, down-regulation of contractile ring contraction involved in cell cycle cytokinesis involved in mitotic cell cycle, down-regulation of cytokinesis, actomyosin ring contraction involved in mitotic cell cycle, down-regulation of mitotic actomyosin contractile ring contraction, downregulation of contractile ring contraction involved in cell cycle cytokinesis involved in mitotic cell cycle, downregulation of cytokinesis, actomyosin ring contraction involved in mitotic cell cycle, downregulation of mitotic actomyosin contractile ring contraction, negative regulation of contractile ring contraction involved in cell cycle cytokinesis involved in mitotic cell cycle, negative regulation of cytokinesis, actomyosin ring contraction involved in mitotic cell cycle, negative regulation of mitotic actomyosin contractile ring constriction, inhibition of contractile ring contraction involved in cell cycle cytokinesis involved in mitotic cell cycle, inhibition of cytokinesis, actomyosin ring contraction involved in mitotic cell cycle, inhibition of mitotic actomyosin contractile ring contraction Relationships: is a type of negative regulation of mitotic cytokinetic process [GO:1903437]; is a type of GO:1903471; negatively regulates mitotic actomyosin contractile ring contraction [GO:1902404]